{
  "gene_symbol": "CDS2",
  "term_id": "GO:0140042",
  "gene_name": "Phosphatidate cytidylyltransferase 2",
  "gene": "UniProtKB:O95674",
  "term_label": "lipid droplet formation"
}